{
  "term_id": "GO:0007423",
  "gene": "UniProtKB:Q13402",
  "term_label": "sensory organ development",
  "gene_name": "Unconventional myosin-VIIa",
  "gene_symbol": "MYO7A"
}